B cell deletion [GO:0002516] (biological process) Sources: GOC:add, GOC:jal, ISBN:0781735149 Definition: The apoptotic death of B cells which is part of B cell tolerance induction. Relationships: is a type of GO:0001783; is a type of apoptotic process involved in development [GO:1902742]; is part of B cell tolerance induction [GO:0002514] Regulation: RO_0002211 by regulation of B cell deletion [GO:0002867]; negatively regulated by negative regulation of B cell deletion [GO:0002868]; positively regulated by positive regulation of B cell deletion [GO:0002869] Subtypes: central B cell deletion [GO:0002342], peripheral B cell deletion [GO:0002454] Also known as: B lymphocyte deletion, B-cell deletion, B-lymphocyte deletion